{
  "gene_symbol": "ZFPM1",
  "term_label": "transcription corepressor activity",
  "gene_name": "Zinc finger protein ZFPM1",
  "term_id": "GO:0003714",
  "gene": "UniProtKB:Q8IX07"
}